cell-cell signaling involved in metanephros development [GO:0072204] (biological process) Definition: Any process that mediates the transfer of information from one cell to another and contributes to the progression of the metanephros over time, from its formation to the mature organ. Also known as: cell-cell signalling involved in metanephros development Relationships: is a type of cell-cell signaling involved in kidney development [GO:0060995]; is part of metanephros development [GO:0001656] Sources: GOC:mtg_kidney_jan10